{
  "gene_symbol": "KIF1B",
  "gene_name": "Kinesin-like protein KIF1B",
  "gene": "UniProtKB:O60333",
  "term_label": "plus-end-directed microtubule motor activity",
  "term_id": "GO:0008574"
}